{
  "gene_name": "Junction plakoglobin",
  "term_id": "GO:0045944",
  "term_label": "positive regulation of transcription by RNA polymerase II",
  "gene": "UniProtKB:P14923",
  "gene_symbol": "JUP"
}